GDP-D-glucose phosphorylase activity [GO:0080048] (molecular function) Also known as: GDP:glucose-1-phosphate guanyltransferase activity, glucose-1-phosphate guanylyltransferase (GDP) activity References: PMID:17462988, PMID:18463094 Definition: Catalysis of the reaction: GDP-alpha-D-glucose + phosphate = alpha-D-glucose-1-phosphate + GDP. Relationships: is_a guanylyltransferase activity [GO:0070568]